{
  "gene": "UniProtKB:Q53QW1",
  "term_id": "UNKNOWN:0003",
  "gene_name": "Testis-expressed protein 44",
  "gene_symbol": "TEX44",
  "term_label": "Unknown cellular component"
}